{
  "gene_symbol": "GRAMD2A",
  "term_id": "GO:0005789",
  "term_label": "endoplasmic reticulum membrane",
  "gene": "UniProtKB:Q8IUY3",
  "gene_name": "GRAM domain-containing protein 2A"
}